{
  "gene": "UniProtKB:O00160",
  "term_id": "GO:0051015",
  "term_label": "actin filament binding",
  "gene_name": "Unconventional myosin-If",
  "gene_symbol": "MYO1F"
}